{
  "term_id": "GO:0005525",
  "gene_symbol": "RAB39B",
  "gene_name": "Ras-related protein Rab-39B",
  "gene": "UniProtKB:Q96DA2",
  "term_label": "GTP binding"
}